{
  "term_id": "UNKNOWN:0001",
  "gene_name": "Acid phosphatase type 7",
  "gene_symbol": "ACP7",
  "term_label": "Unknown molecular function",
  "gene": "UniProtKB:Q6ZNF0"
}